{
  "gene": "UniProtKB:Q8TEY5",
  "gene_name": "Cyclic AMP-responsive element-binding protein 3-like protein 4",
  "term_id": "GO:0006357",
  "gene_symbol": "CREB3L4",
  "term_label": "regulation of transcription by RNA polymerase II"
}